{
  "gene_name": "BMP-2-inducible protein kinase",
  "term_label": "nucleus",
  "term_id": "GO:0005634",
  "gene": "UniProtKB:Q9NSY1",
  "gene_symbol": "BMP2K"
}